{
  "gene": "UniProtKB:Q9NQV8",
  "gene_name": "PR domain zinc finger protein 8",
  "term_id": "GO:0014003",
  "gene_symbol": "PRDM8",
  "term_label": "oligodendrocyte development"
}